{
  "term_id": "GO:0031695",
  "gene": "UniProtKB:P51693",
  "gene_name": "Amyloid beta precursor like protein 1",
  "gene_symbol": "APLP1",
  "term_label": "alpha-2B adrenergic receptor binding"
}